membrane raft assembly [GO:0001765] (biological process) Also known as: lipid raft assembly, lipid raft formation, membrane raft formation Definition: The aggregation, arrangement and bonding together of a set of components to form a membrane raft, a small (10-200 nm), heterogeneous, highly dynamic, sterol- and sphingolipid-enriched membrane domains that compartmentalizes cellular processes. Subtypes: plasma membrane raft assembly [GO:0044854] References: PMID:12648772, PMID:12803918, PMID:16645198 Relationships: is a type of membrane raft organization [GO:0031579]; is a type of membrane assembly [GO:0071709]